{
  "term_id": "GO:0008195",
  "term_label": "phosphatidate phosphatase activity",
  "gene_symbol": "LPIN1",
  "gene_name": "Phosphatidate phosphatase LPIN1",
  "gene": "UniProtKB:Q14693"
}